{
  "term_id": "GO:0000813",
  "gene_name": "Ubiquitin-associated protein 1-like",
  "term_label": "ESCRT I complex",
  "gene": "UniProtKB:F5GYI3",
  "gene_symbol": "UBAP1L"
}